lipopolysaccharide localization to cell outer membrane [GO:0140334] (biological process) References: PMID:24639492 Definition: A process in which a lipopolysaccharide is transported to the cell outer membrane. Also known as: LPS localization to cell outer membrane Relationships: is a type of lipid localization [GO:0010876]; is_a localization within membrane [GO:0051668]